{
  "term_label": "tubulin complex assembly",
  "term_id": "GO:0007021",
  "gene": "UniProtKB:O75347",
  "gene_symbol": "TBCA",
  "gene_name": "Tubulin-specific chaperone A"
}